{
  "term_label": "Unknown biological process",
  "gene_symbol": "WDR93",
  "gene": "UniProtKB:Q6P2C0",
  "term_id": "UNKNOWN:0002",
  "gene_name": "WD repeat-containing protein 93"
}